{
  "term_label": "Unknown cellular component",
  "gene_name": "Putative ankyrin repeat domain-containing protein 19",
  "gene_symbol": "ANKRD19P",
  "gene": "UniProtKB:Q9H560",
  "term_id": "UNKNOWN:0003"
}